translocation of molecules into symbiont [GO:0051862] (biological process) Definition: The directed movement of molecule(s) produced by an organism to a location inside the symbiont organism. The symbiont is defined as the smaller of the organisms involved in a symbiotic interaction. Also known as: transport of molecules into symbiont Subtypes: translocation of peptides or proteins into symbiont [GO:0051844] Relationships: is a type of GO:0051702 Sources: GOC:cc